penetration hypha formation [GO:0075201] (biological process) Regulation: RO_0002211 by GO:0075202; positively regulated by positive regulation of penetration hypha formation [GO:0075203] Definition: The assembly by the symbiont of a threadlike, tubular structure, which may contain multiple nuclei and may or may not be divided internally by septa or cross-walls, for the purpose of penetration into its host organism. In the case of an appressorium existing, this term is defined in further details as the process in which the symbiont penetration peg expands to form a hypha which traverses the epidermal cell and emerges into the intercellular space of the mesophyll tissue. The host is defined as the larger of the organisms involved in a symbiotic interaction. References: PMID:26441323 Sources: GOC:pamgo_curators Relationships: is a type of formation of infection structure [GO:0075015] Also known as: formation of symbiont penetration hypha for entry into host, symbiont penetration hypha formation for entry into host Note: Note that this term should not be used to annotate gene products of the host. It should only be used to annotate those gene products from the symbiont involved in this process.